{
  "term_id": "GO:0036064",
  "gene_name": "Polyglutamylase complex subunit TTLL1",
  "gene_symbol": "TTLL1",
  "gene": "UniProtKB:O95922",
  "term_label": "ciliary basal body"
}